smooth muscle cell differentiation involved in prostate glandular acinus development [GO:0060530] (biological process) Relationships: is a type of developmental process involved in reproduction [GO:0003006]; is a type of smooth muscle cell differentiation [GO:0051145]; is part of prostate glandular acinus development [GO:0060525] References: PMID:18977204 Sources: GOC:dph Definition: The process in which a relatively unspecialized cell acquires specialized features of a smooth muscle cell of the prostate glandular acinus.